{
  "term_label": "Unknown cellular component",
  "gene": "UniProtKB:P15531",
  "gene_symbol": "NME1",
  "gene_name": "Nucleoside diphosphate kinase A",
  "term_id": "UNKNOWN:0003"
}